{
  "gene_symbol": "RIPPLY2",
  "gene": "UniProtKB:Q5TAB7",
  "term_id": "UNKNOWN:0001",
  "gene_name": "Protein ripply2",
  "term_label": "Unknown molecular function"
}